{
  "gene_name": "Mitochondrial nicotinamide adenine dinucleotide transporter SLC25A52",
  "gene": "UniProtKB:Q3SY17",
  "term_id": "GO:1990549",
  "gene_symbol": "SLC25A52",
  "term_label": "mitochondrial NAD transmembrane transport"
}